{
  "gene_symbol": "Q6ZVL8",
  "term_id": "UNKNOWN:0003",
  "gene_name": "Putative uncharacterized protein FLJ42384",
  "term_label": "Unknown cellular component",
  "gene": "UniProtKB:Q6ZVL8"
}